histamine catabolic process [GO:0001695] (biological process) Definition: The chemical reactions and pathways resulting in the breakdown of histamine, a physiologically active amine, found in plant and animal tissue and released from mast cells as part of an allergic reaction in humans. Sources: GOC:jl, ISBN:0395825172 Also known as: histamine breakdown, histamine catabolism, histamine degradation Relationships: is a type of histamine metabolic process [GO:0001692]; is_a biogenic amine catabolic process [GO:0042402]; is a type of GO:0052805